facial nerve development [GO:0021561] (biological process) Relationships: is a type of GO:0021545; is part of preganglionic parasympathetic fiber development [GO:0021783] Also known as: cranial nerve 7 development, cranial nerve VII development, CN VII development Sources: GOC:cls, GOC:dgh, GOC:dph, GOC:jid, GO_REF:0000021 Definition: The process whose specific outcome is the progression of the facial nerve over time, from its formation to the mature structure. This sensory and motor nerve supplies the muscles of facial expression and the expression and taste at the anterior two-thirds of the tongue. The principal branches are the superficial ophthalmic, buccal, palatine and hyomandibular. The main trunk synapses within pterygopalatine ganglion in the parotid gland and this ganglion then gives off nerve branches which supply the lacrimal gland and the mucous secreting glands of the nasal and oral cavities.